response to carbon monoxide [GO:0034465] (biological process) Sources: GOC:ecd Subtypes: GO:0071245 Relationships: is_a response to oxygen-containing compound [GO:1901700] Definition: Any process that results in a change in state or activity of a cell or an organism (in terms of movement, secretion, enzyme production, gene expression, etc.) as a result of a carbon monoxide (CO) stimulus.